{
  "gene_name": "Tubulin beta-2B chain",
  "gene_symbol": "TUBB2B",
  "term_id": "GO:0001764",
  "term_label": "neuron migration",
  "gene": "UniProtKB:Q9BVA1"
}